regulation of CAMKK-AMPK signaling cascade [GO:1905289] (biological process) Definition: Any process that modulates the frequency, rate or extent of CAMKK-AMPK signaling cascade. Relationships: is a type of GO:0050848; regulates GO:0061762 References: PMID:22128786 Sources: GOC:TermGenie, GO_REF:0000058 Subtypes: negative regulation of CAMKK-AMPK signaling cascade [GO:1905290], GO:1905291 Also known as: regulation of stress-activated AMP-activated protein kinase signaling cascade